{
  "gene_symbol": "IGHG3",
  "term_id": "GO:0006958",
  "term_label": "complement activation, classical pathway",
  "gene": "UniProtKB:P01860",
  "gene_name": "Immunoglobulin heavy constant gamma 3"
}